{
  "term_label": "double-strand break repair via break-induced replication",
  "gene": "UniProtKB:Q4G0Z9",
  "gene_name": "Minichromosome maintenance domain-containing protein 2",
  "gene_symbol": "MCMDC2",
  "term_id": "GO:0000727"
}